{
  "gene": "UniProtKB:Q5VWW1",
  "term_label": "synaptic cleft",
  "gene_name": "Complement C1q-like protein 3",
  "gene_symbol": "C1QL3",
  "term_id": "GO:0043083"
}